{
  "gene": "UniProtKB:Q8IXF0",
  "term_label": "DNA-binding transcription factor activity, RNA polymerase II-specific",
  "term_id": "GO:0000981",
  "gene_name": "Neuronal PAS domain-containing protein 3",
  "gene_symbol": "NPAS3"
}